regulation of L-proline catabolic process to L-glutamate [GO:2001156] (biological process) Also known as: regulation of proline catabolic process to glutamate, regulation of proline breakdown to glutamate, regulation of proline degradation to glutamate, regulation of proline oxidation Definition: Any process that modulates the frequency, rate or extent of L-proline catabolic process to L-glutamate. Sources: GOC:obol Relationships: is a type of regulation of catabolic process [GO:0009894]; is a type of regulation of glutamate metabolic process [GO:2000211]; is a type of regulation of L-proline metabolic process [GO:2000214]; regulates L-proline catabolic process to L-glutamate [GO:0010133] Subtypes: GO:2001157, positive regulation of L-proline catabolic process to L-glutamate [GO:2001158]